{
  "gene_symbol": "DVL1P1",
  "gene_name": "Putative segment polarity protein dishevelled homolog DVL1P1",
  "term_label": "canonical Wnt signaling pathway",
  "gene": "UniProtKB:P54792",
  "term_id": "GO:0060070"
}